{
  "term_id": "GO:0035032",
  "term_label": "phosphatidylinositol 3-kinase complex, class III",
  "gene_symbol": "ATG14",
  "gene_name": "Beclin 1-associated autophagy-related key regulator",
  "gene": "UniProtKB:Q6ZNE5"
}